{
  "term_label": "Golgi apparatus",
  "gene_name": "Protein CLEC16A",
  "term_id": "GO:0005794",
  "gene": "UniProtKB:Q2KHT3",
  "gene_symbol": "CLEC16A"
}